{
  "gene_name": "CAAX prenyl protease 2",
  "gene": "UniProtKB:Q9Y256",
  "gene_symbol": "RCE1",
  "term_id": "GO:0071586",
  "term_label": "CAAX-box protein processing"
}